{
  "gene": "UniProtKB:A4D2H0",
  "gene_name": "cTAGE family member 15",
  "term_id": "GO:0070971",
  "gene_symbol": "CTAGE15",
  "term_label": "endoplasmic reticulum exit site"
}